{
  "gene_symbol": "CASP8",
  "term_id": "GO:0043525",
  "gene_name": "Caspase-8",
  "gene": "UniProtKB:Q14790",
  "term_label": "positive regulation of neuron apoptotic process"
}